{
  "gene_symbol": "CDK4",
  "term_id": "GO:0005737",
  "gene_name": "Cyclin-dependent kinase 4",
  "gene": "UniProtKB:P11802",
  "term_label": "cytoplasm"
}